{
  "gene_name": "Chitobiosyldiphosphodolichol beta-mannosyltransferase",
  "term_id": "UNKNOWN:0002",
  "term_label": "Unknown biological process",
  "gene_symbol": "ALG1",
  "gene": "UniProtKB:Q9BT22"
}